methionine-importing complex [GO:1902509] (CC) Subtypes: GO:1990197 Relationships: is a type of GO:1902495 Also known as: methionine importer complex, methionine importing complex Definition: A protein complex which is capable of methionine-importing activity. References: PMID:23748165 Sources: GOC:TermGenie, GOC:pr